{
  "gene_name": "Synaptotagmin-11",
  "term_id": "GO:0000149",
  "term_label": "SNARE binding",
  "gene": "UniProtKB:Q9BT88",
  "gene_symbol": "SYT11"
}